{
  "gene_name": "Pachytene checkpoint protein 2 homolog",
  "gene_symbol": "TRIP13",
  "term_label": "reciprocal meiotic recombination",
  "gene": "UniProtKB:Q15645",
  "term_id": "GO:0007131"
}